{
  "term_label": "nervous system development",
  "gene_name": "Palmitoyl-protein thioesterase 1",
  "gene_symbol": "PPT1",
  "gene": "UniProtKB:P50897",
  "term_id": "GO:0007399"
}